thiamine pyrophosphate binding [GO:0030976] (molecular function) Definition: Binding to thiamine pyrophosphate, the diphosphoric ester of thiamine. Acts as a coenzyme of several (de)carboxylases, transketolases, and alpha-oxoacid dehydrogenases. Also known as: TPP binding, aneurine pyrophosphate binding, cocarboxylase binding, diphosphothiamin binding, thiamin pyrophosphate binding Sources: GOC:mlg Relationships: is a type of vitamin binding [GO:0019842]; is a type of anion binding [GO:0043168]; is a type of cation binding [GO:0043169]; is a type of GO:0050997; is a type of GO:1901363; is a type of sulfur compound binding [GO:1901681]